{
  "term_label": "positive regulation of transcription by RNA polymerase II",
  "gene": "UniProtKB:Q14686",
  "gene_symbol": "NCOA6",
  "gene_name": "Nuclear receptor coactivator 6",
  "term_id": "GO:0045944"
}